{
  "gene_symbol": "LOXL2",
  "gene": "UniProtKB:Q9Y4K0",
  "term_id": "GO:0004720",
  "gene_name": "Lysyl oxidase homolog 2",
  "term_label": "protein-lysine 6-oxidase activity"
}